{
  "gene": "UniProtKB:Q9N2J8",
  "term_id": "UNKNOWN:0001",
  "term_label": "Unknown molecular function",
  "gene_symbol": "Q9N2J8",
  "gene_name": "HERV-H_2q24.1 provirus ancestral Env polyprotein"
}